host cell endosome lumen [GO:0072493] (cellular component) Also known as: host endosome lumen Relationships: is a type of host cell cytoplasm part [GO:0033655]; is part of host cell endosome [GO:0044174] Sources: GOC:ecd Definition: The volume enclosed by the membranes of the host cell endosome.